{
  "gene_symbol": "NLRP12",
  "gene_name": "NACHT, LRR and PYD domains-containing protein 12",
  "term_label": "cytoplasm",
  "term_id": "GO:0005737",
  "gene": "UniProtKB:P59046"
}